{
  "gene_symbol": "P2RY13",
  "term_id": "GO:0007186",
  "gene": "UniProtKB:Q9BPV8",
  "term_label": "G protein-coupled receptor signaling pathway",
  "gene_name": "P2Y purinoceptor 13"
}